{
  "term_label": "protein-folding chaperone binding",
  "term_id": "GO:0051087",
  "gene": "UniProtKB:O75190",
  "gene_symbol": "DNAJB6",
  "gene_name": "DnaJ homolog subfamily B member 6"
}